{
  "gene_symbol": "LCE5A",
  "term_label": "Unknown cellular component",
  "gene": "UniProtKB:Q5TCM9",
  "gene_name": "Late cornified envelope protein 5A",
  "term_id": "UNKNOWN:0003"
}